{
  "term_id": "UNKNOWN:0001",
  "gene": "UniProtKB:A6NDB9",
  "gene_name": "Paralemmin-3",
  "gene_symbol": "PALM3",
  "term_label": "Unknown molecular function"
}